{
  "term_label": "creatine kinase activity",
  "gene_name": "Creatine kinase U-type, mitochondrial",
  "term_id": "GO:0004111",
  "gene": "UniProtKB:P12532",
  "gene_symbol": "CKMT1A"
}